diolein transacylation activity [GO:0051265] (molecular function) References: PMID:15364929 Sources: GOC:ai Also known as: DOG transacylation, acyl-CoA-independent diolein transacylation, dioleoylglycerol O-acyltransferase activity, dioleoylglycerol transacylase activity Definition: Catalysis of the reaction: diolein + mono-olein = triolein + glycerol. Mono-olein, also known as mono-oleoylglycerol, is the monoglyceride formed from oleic acid, 9-octodecenoic acid; diolein is also known as dioleoylglycerol, and triolein as trioleoylglycerol and olein. Relationships: is a type of acylglycerol O-acyltransferase activity [GO:0016411]